{
  "term_id": "GO:0005184",
  "gene_symbol": "NMB",
  "gene": "UniProtKB:P08949",
  "gene_name": "Neuromedin-B",
  "term_label": "neuropeptide hormone activity"
}